{
  "term_id": "UNKNOWN:0003",
  "gene": "UniProtKB:O95628",
  "term_label": "Unknown cellular component",
  "gene_symbol": "CNOT4",
  "gene_name": "CCR4-NOT transcription complex subunit 4"
}